nuclear export signal receptor activity [GO:0005049] (molecular function) Definition: Combining with a nuclear export signal (NES) on a cargo to be transported, to mediate transport of a the cargo through the nuclear pore, from the nuclear lumen to the cytoplasm. The cargo can be either a RNA or a protein. References: PMID:11743003, PMID:25802992, PMID:28713609 Sources: GOC:bf, GOC:mah, GOC:pg, GOC:vw, Wikipedia:Nuclear_transport Also known as: NES receptor, importin-alpha export receptor activity, exportin activity, importin-alpha binding Relationships: is a type of nucleocytoplasmic carrier activity [GO:0140142]; is part of nuclear export [GO:0051168]